{
  "term_label": "chromatin remodeling",
  "gene_name": "Chromatin accessibility complex protein 1",
  "gene_symbol": "CHRAC1",
  "gene": "UniProtKB:Q9NRG0",
  "term_id": "GO:0006338"
}